{
  "gene_name": "Telomerase protein component 1",
  "term_label": "telomerase holoenzyme complex",
  "gene": "UniProtKB:Q99973",
  "gene_symbol": "TEP1",
  "term_id": "GO:0005697"
}